{
  "gene_name": "Potassium voltage-gated channel subfamily C member 1",
  "term_id": "GO:0032590",
  "term_label": "dendrite membrane",
  "gene_symbol": "KCNC1",
  "gene": "UniProtKB:P48547"
}